{
  "gene_symbol": "ATG4C",
  "term_label": "mitophagy",
  "term_id": "GO:0000423",
  "gene": "UniProtKB:Q96DT6",
  "gene_name": "Cysteine protease ATG4C"
}